{
  "gene_symbol": "MYO1B",
  "term_label": "microvillus",
  "gene": "UniProtKB:O43795",
  "term_id": "GO:0005902",
  "gene_name": "Unconventional myosin-Ib"
}